{
  "gene_name": "Asporin",
  "term_id": "GO:0005615",
  "gene_symbol": "ASPN",
  "gene": "UniProtKB:Q9BXN1",
  "term_label": "extracellular space"
}